{
  "gene_symbol": "ATG101",
  "term_id": "GO:0000045",
  "term_label": "autophagosome assembly",
  "gene_name": "Autophagy-related protein 101",
  "gene": "UniProtKB:Q9BSB4"
}